{
  "term_label": "short-chain fatty acyl-CoA dehydrogenase activity",
  "term_id": "GO:0016937",
  "gene_symbol": "ACADS",
  "gene_name": "Short-chain specific acyl-CoA dehydrogenase, mitochondrial",
  "gene": "UniProtKB:P16219"
}